intrinsic apoptotic signaling pathway in response to hypoxia [GO:1990144] (biological process) Regulation: regulated by regulation of hypoxia-induced intrinsic apoptotic signaling pathway [GO:1903297]; negatively regulated by GO:1903298 Definition: The series of molecular signals in which an intracellular signal is conveyed to trigger the apoptotic death of a cell. The pathway is induced in response to hypoxia (lowered oxygen tension). Hypoxia, defined as a decline in O2 levels below normoxic levels of 20.8 - 20.95%, results in metabolic adaptation at both the cellular and organismal level. The pathway ends when the execution phase of apoptosis is triggered. Relationships: is_a intrinsic apoptotic signaling pathway [GO:0097193]; is part of cellular response to hypoxia [GO:0071456] References: PMID:20436456 Sources: GOC:BHF, GOC:mtg_apoptosis, GOC:rl